{
  "term_label": "small GTPase-mediated signal transduction",
  "gene_name": "Guanine nucleotide exchange factor VAV2",
  "gene_symbol": "VAV2",
  "term_id": "GO:0007264",
  "gene": "UniProtKB:P52735"
}